{
  "gene_name": "Glycerol-3-phosphate acyltransferase 2, mitochondrial",
  "gene": "UniProtKB:Q6NUI2",
  "term_label": "glycerol-3-phosphate O-acyltransferase activity",
  "term_id": "GO:0004366",
  "gene_symbol": "GPAT2"
}